{
  "term_id": "GO:0050982",
  "gene_symbol": "PIEZO2",
  "term_label": "detection of mechanical stimulus",
  "gene": "UniProtKB:Q9H5I5",
  "gene_name": "Piezo-type mechanosensitive ion channel component 2"
}